{
  "gene": "UniProtKB:Q7RTU3",
  "gene_name": "Oligodendrocyte transcription factor 3",
  "gene_symbol": "OLIG3",
  "term_label": "DNA-binding transcription factor activity, RNA polymerase II-specific",
  "term_id": "GO:0000981"
}